{
  "gene": "UniProtKB:Q6P582",
  "gene_name": "Mitotic-spindle organizing protein 2A",
  "term_id": "GO:0005819",
  "gene_symbol": "MZT2A",
  "term_label": "spindle"
}